alpha-linked polysaccharide catabolism to maltotriose [GO:0052786] (biological process) Relationships: is a type of GO:0000272 References: PMID:7511484, PMID:9406414 Sources: GOC:mengo_curators Definition: The breakdown of large alpha-linked polysaccharides by hydrolysis of (1->4)-alpha-D-glucosidic linkages to yield maltotriose. Also known as: alpha-amylase-mediated polysaccharide catabolism, producing maltotriose, maltotriose-forming alpha-amylase activity